{
  "term_id": "GO:0030395",
  "gene": "UniProtKB:Q96DT0",
  "gene_symbol": "LGALS12",
  "term_label": "lactose binding",
  "gene_name": "Galectin-12"
}